alpha-latrotoxin receptor binding [GO:0061761] (molecular function) Definition: Binding to an alpha-latrotoxin receptor. References: PMID:21724987 Sources: GOC:dph Also known as: lasso receptor binding, latrophilin binding Relationships: is a type of G protein-coupled receptor binding [GO:0001664]